{
  "gene": "UniProtKB:Q9HA77",
  "term_id": "GO:0005524",
  "gene_name": "Probable cysteine--tRNA ligase, mitochondrial",
  "gene_symbol": "CARS2",
  "term_label": "ATP binding"
}